ABC-type nitrate transporter activity [GO:0015414] (molecular function) Relationships: is a type of GO:0015112; is a type of ABC-type transporter activity [GO:0140359] Sources: RHEA:13181 Also known as: nitrate ABC transporter, ATPase-coupled nitrate transmembrane transporter activity, nitrate transmembrane-transporting ATPase activity, nitrate transporting ATPase activity, nitrate-transporting ATPase activity Definition: Enables the transfer of a solute or solutes from one side of a membrane to the other according to the reaction: ATP + H2O + nitrate(out) = ADP + phosphate + nitrate(in).